negative regulation of metanephric S-shaped body morphogenesis [GO:2000005] (biological process) Sources: GOC:mtg_kidney_jan10, GOC:obol, GOC:yaf Definition: Any process that stops, prevents, or reduces the frequency, rate or extent of metanephric S-shaped body morphogenesis. Relationships: is a type of negative regulation of developmental process [GO:0051093]; is a type of regulation of metanephric S-shaped body morphogenesis [GO:2000004]; negatively regulates metanephric S-shaped body morphogenesis [GO:0072284]